{
  "gene_symbol": "SEC14L4",
  "term_id": "GO:0005737",
  "gene_name": "SEC14-like protein 4",
  "gene": "UniProtKB:Q9UDX3",
  "term_label": "cytoplasm"
}